{
  "term_label": "positive regulation of filopodium assembly",
  "gene_symbol": "PALM",
  "term_id": "GO:0051491",
  "gene_name": "Paralemmin-1",
  "gene": "UniProtKB:O75781"
}